epicardium-derived cardiac endothelial cell differentiation [GO:0003349] (biological process) Relationships: is a type of cardiac endothelial cell differentiation [GO:0003348] References: PMID:18722343 Sources: GOC:dph Definition: The process in which an epicardial cell acquires the specialized structural and/or functional features of a cardiac endothelial cell.